mesonephric capsule development [GO:0061285] (biological process) Definition: The progression of the mesonephric capsule over time, from its formation to the mature structure. The mesonephric capsule is the tough fibrous layer surrounding the mesonephros, covered in a thick layer of perinephric adipose tissue. Sources: GOC:mtg_kidney_jan10 Relationships: is a type of renal capsule development [GO:0072127]; is part of mesonephros development [GO:0001823]